{
  "term_id": "GO:0055037",
  "gene_symbol": "RAB25",
  "gene": "UniProtKB:P57735",
  "term_label": "recycling endosome",
  "gene_name": "Ras-related protein Rab-25"
}